{
  "gene_symbol": "YJEFN3",
  "gene_name": "YjeF N-terminal domain-containing protein 3",
  "term_id": "UNKNOWN:0002",
  "term_label": "Unknown biological process",
  "gene": "UniProtKB:A6XGL0"
}